{
  "term_id": "GO:0071568",
  "gene": "UniProtKB:Q9Y3C8",
  "gene_symbol": "UFC1",
  "gene_name": "Ubiquitin-fold modifier-conjugating enzyme 1",
  "term_label": "UFM1 transferase activity"
}